hydrolase activity, acting on acid anhydrides, in phosphorus-containing anhydrides [GO:0016818] (molecular function) Relationships: is_a hydrolase activity, acting on acid anhydrides [GO:0016817] Sources: GOC:jl Definition: Catalysis of the hydrolysis of any acid anhydride which contains phosphorus. Subtypes: GO:0016462, dihydroneopterin monophosphate phosphatase activity [GO:0019176], nucleoside phosphoacylhydrolase activity [GO:0033974], phosphocholine hydrolase activity [GO:0044606], 5'-acylphosphoadenosine hydrolase activity [GO:0047586], trimetaphosphatase activity [GO:0050351], cyclic-GMP-AMP hydrolase activity [GO:0106177], N6-methyl-(d)ATP hydrolase activity [GO:0106431], O6-methyl-dGTP hydrolase activity [GO:0106433], RNA NAD+-cap (NAD+-forming) hydrolase activity [GO:0110152]